{
  "term_id": "GO:0042127",
  "gene_name": "Transforming growth factor beta-2 proprotein",
  "gene_symbol": "TGFB2",
  "term_label": "regulation of cell population proliferation",
  "gene": "UniProtKB:P61812"
}